venom-mediated disruption of extracellular matrix in another organism [GO:0044523] (biological process) Definition: A process that begins with venom being forced into an organism by the bite or sting of another organism, damaging the extracellular matrix of a cell. Also known as: envenomation resulting in damage of muscle extracellular matrix causing muscle necrosis in other organism, envenomation resulting in damage of muscle extracellular matrix in another organism, envenomation resulting in damage of muscle extracellular matrix in other organism Relationships: is a type of venom-mediated disruption of anatomical structure in another organism [GO:0140138] References: PMID:20398688, PMID:21150580, PMID:33460638 Sources: GOC:fj, GOC:jl